{
  "gene_name": "Oncoprotein-induced transcript 3 protein",
  "gene": "UniProtKB:Q8WWZ8",
  "gene_symbol": "OIT3",
  "term_id": "GO:0005615",
  "term_label": "extracellular space"
}